{
  "gene_name": "Keratin, type II cytoskeletal 75",
  "term_label": "keratinization",
  "term_id": "GO:0031424",
  "gene": "UniProtKB:O95678",
  "gene_symbol": "KRT75"
}